{
  "gene": "UniProtKB:Q9NWB1",
  "gene_name": "RNA binding protein fox-1 homolog 1",
  "gene_symbol": "RBFOX1",
  "term_id": "GO:0003729",
  "term_label": "mRNA binding"
}